neuromelanin biosynthetic process [GO:0036489] (biological process) Definition: The chemical reactions and pathways resulting in the formation of neuromelanin. Neuromelanin is a polymer of 5,6-dihydroxyindole monomers. Relationships: is_a macromolecule biosynthetic process [GO:0009059] Also known as: neuromelanin anabolism, neuromelanin biosynthesis, neuromelanin formation, neuromelanin synthesis Sources: GOC:PARL, GOC:bf, Wiki:Neuromelanin